{
  "gene": "UniProtKB:Q2QD12",
  "term_id": "GO:0046872",
  "gene_name": "Ribulose-phosphate 3-epimerase-like protein 1",
  "gene_symbol": "RPEL1",
  "term_label": "metal ion binding"
}